opsin transport [GO:0036372] (biological process) Definition: The directed movement of an opsin (a G protein-coupled receptor of photoreceptor cells) into, out of or within a cell, or between cells, or within a multicellular organism by means of some agent such as a transporter or pore. Also known as: ciliary transport of opsin References: PMID:20238016, PMID:22855808 Sources: GOC:atm Relationships: is a type of GO:0015031